{
  "gene_symbol": "ABHD14B",
  "gene": "UniProtKB:Q96IU4",
  "term_label": "cytoplasm",
  "gene_name": "Putative protein-lysine deacylase ABHD14B",
  "term_id": "GO:0005737"
}